{
  "gene": "UniProtKB:Q9UHW9",
  "gene_name": "Solute carrier family 12 member 6",
  "gene_symbol": "SLC12A6",
  "term_id": "GO:0055064",
  "term_label": "chloride ion homeostasis"
}